ornithine biosynthetic process [GO:0006592] (biological process) Also known as: ornithine anabolism, ornithine biosynthesis, ornithine formation, ornithine synthesis Definition: The chemical reactions and pathways resulting in the formation of ornithine, an amino acid only rarely found in proteins, but which is important in living organisms as an intermediate in the reactions of the urea cycle and in arginine biosynthesis. Relationships: is_a ornithine metabolic process [GO:0006591]; is a type of non-proteinogenic amino acid biosynthetic process [GO:0170043]; is a type of alpha-amino acid biosynthetic process [GO:1901607] Sources: GOC:jl, ISBN:0192801023